{
  "term_id": "GO:0005184",
  "term_label": "neuropeptide hormone activity",
  "gene_name": "Oxytocin-neurophysin 1",
  "gene_symbol": "OXT",
  "gene": "UniProtKB:P01178"
}